{
  "gene": "UniProtKB:Q6NZ67",
  "gene_name": "Mitotic-spindle organizing protein 2B",
  "term_label": "Unknown biological process",
  "gene_symbol": "MZT2B",
  "term_id": "UNKNOWN:0002"
}